{
  "term_label": "Unknown biological process",
  "gene_symbol": "LINC01558",
  "gene_name": "Uncharacterized protein encoded by LINC01558",
  "term_id": "UNKNOWN:0002",
  "gene": "UniProtKB:Q9Y6Z2"
}